4-hydroxybenzaldehyde dehydrogenase (NAD+) activity [GO:0018484] (molecular function) Also known as: 3-hydroxybenzaldehyde:NAD+ oxidoreductase activity, p-hydroxybenzaldehyde dehydrogenase activity Sources: EC:1.2.1.64 Relationships: is a type of aldehyde dehydrogenase (NAD+) activity [GO:0004029] Definition: Catalysis of the reaction: 4-hydroxybenzaldehyde + NAD+ + H2O = 4-hydroxybenzoate + NADH + H+.